{
  "gene": "UniProtKB:Q15759",
  "term_label": "protein serine/threonine kinase activity",
  "gene_name": "Mitogen-activated protein kinase 11",
  "term_id": "GO:0004674",
  "gene_symbol": "MAPK11"
}